{
  "gene_symbol": "CA5A",
  "gene": "UniProtKB:P35218",
  "term_label": "carbonate dehydratase activity",
  "gene_name": "Carbonic anhydrase 5A, mitochondrial",
  "term_id": "GO:0004089"
}